{
  "gene_symbol": "PI4KAP2",
  "gene": "UniProtKB:A4QPH2",
  "gene_name": "Putative phosphatidylinositol 4-kinase alpha-like protein P2",
  "term_label": "Unknown biological process",
  "term_id": "UNKNOWN:0002"
}